{
  "gene": "UniProtKB:P58397",
  "gene_symbol": "ADAMTS12",
  "term_id": "GO:0006508",
  "term_label": "proteolysis",
  "gene_name": "A disintegrin and metalloproteinase with thrombospondin motifs 12"
}